{
  "gene_symbol": "CENPN",
  "gene": "UniProtKB:Q96H22",
  "term_label": "nucleoplasm",
  "term_id": "GO:0005654",
  "gene_name": "Centromere protein N"
}